{
  "gene_name": "Angiopoietin-related protein 3",
  "term_id": "GO:0004859",
  "gene": "UniProtKB:Q9Y5C1",
  "term_label": "phospholipase inhibitor activity",
  "gene_symbol": "ANGPTL3"
}